{
  "term_id": "UNKNOWN:0003",
  "gene_name": "GTPase IMAP family member 5",
  "gene": "UniProtKB:Q96F15",
  "term_label": "Unknown cellular component",
  "gene_symbol": "GIMAP5"
}